hydroxypyruvate reductase (NADPH) activity [GO:0120509] (molecular function) Sources: RHEA:18657 Relationships: is a type of hydroxypyruvate reductase [NAD(P)H] activity [GO:0016618] Definition: Catalysis of the reaction: (R)-glycerate + NADP+ = 3-hydroxypyruvate + NADPH + H+.